cyclohexane-1,3-dione hydrolase activity [GO:0047796] (molecular function) Sources: EC:3.7.1.10, RHEA:16473 Also known as: 1,3-cyclohexanedione hydrolase activity, cyclohexane-1,3-dione acylhydrolase (decyclizing) Definition: Catalysis of the reaction: cyclohexane-1,3-dione + H2O = 5-oxohexanoate + H+. Relationships: is_a hydrolase activity, acting on acid carbon-carbon bonds, in ketonic substances [GO:0016823]